negative regulation of heterochromatin formation [GO:0031452] (biological process) Subtypes: negative regulation of regulatory ncRNA-mediated heterochromatin formation [GO:0060906], negative regulation of silent mating-type cassette heterochromatin formation [GO:0061186], GO:0061188, negative regulation of DNA methylation-dependent heterochromatin formation [GO:0090310] Definition: Any process that stops, prevents, or reduces the frequency, rate or extent of heterochromatin formation. References: PMID:16855380 Also known as: chromatin decompaction, chromatin decondensation, down regulation of heterochromatin formation, down-regulation of heterochromatin formation, downregulation of heterochromatin formation, negative regulation of heterochromatin assembly, inhibition of heterochromatin formation Relationships: is a type of positive regulation of gene expression [GO:0010628]; is a type of regulation of heterochromatin formation [GO:0031445]; is a type of GO:1905268; negatively regulates heterochromatin formation [GO:0031507]